F-9775B biosynthetic process [GO:1900614] (biological process) Regulation: regulated by regulation of F-9775B biosynthetic process [GO:1900675]; RO_0002212 by negative regulation of F-9775B biosynthetic process [GO:1900676]; positively regulated by positive regulation of F-9775B biosynthetic process [GO:1900677] Sources: GOC:TermGenie, GOC:di Also known as: F-9775B anabolism, F-9775B biosynthesis, F-9775B formation, F-9775B synthesis Relationships: is_a polyketide biosynthetic process [GO:0030639]; is a type of phenol-containing compound biosynthetic process [GO:0046189] Definition: The chemical reactions and pathways resulting in the formation of F-9775B.